{
  "gene": "UniProtKB:P30622",
  "gene_symbol": "CLIP1",
  "gene_name": "CAP-Gly domain-containing linker protein 1",
  "term_id": "GO:0005634",
  "term_label": "nucleus"
}